{
  "gene_symbol": "SMCHD1",
  "gene_name": "Structural maintenance of chromosomes flexible hinge domain-containing protein 1",
  "gene": "UniProtKB:A6NHR9",
  "term_label": "Unknown biological process",
  "term_id": "UNKNOWN:0002"
}